{
  "gene_symbol": "FGF17",
  "gene": "UniProtKB:O60258",
  "gene_name": "Fibroblast growth factor 17",
  "term_id": "GO:0005111",
  "term_label": "type 2 fibroblast growth factor receptor binding"
}